synaptonemal structure [GO:0099086] (cellular component) Definition: A proteinaceous scaffold found between homologous chromosomes during meiosis. Sources: GOC:elh, GOC:vw Relationships: is a type of cellular anatomical structure [GO:0110165]; is part of GO:0000794 Subtypes: synaptonemal complex [GO:0000795], linear element [GO:0030998]